Wnt signaling pathway, planar cell polarity pathway [GO:0060071] (biological process) Regulation: negatively regulated by negative regulation of Wnt signaling pathway, planar cell polarity pathway [GO:0141113]; regulated by regulation of Wnt signaling pathway, planar cell polarity pathway [GO:2000095]; positively regulated by positive regulation of Wnt signaling pathway, planar cell polarity pathway [GO:2000096] References: PMID:11532397, PMID:25349257, PMID:28293032, PMID:37804416 Subtypes: regulation of cytoskeleton polarization involved in growth plate cartilage chondrocyte division [GO:0003427], planar cell polarity pathway involved in cardiac muscle cell fate commitment [GO:0061345] Relationships: is a type of non-canonical Wnt signaling pathway [GO:0035567] Definition: A type of non-canonical Wnt signaling pathway in which Wnt binding to its receptor on the surface of a target cell results in the activation small G proteins such as Rho, Rac, and Cdc42 which, in turn activate effectors, including C-Jun N-terminal kinase (JNK) and Rho kinase (Rok). The signaling ends with change in the transcription of target genes and/or reorganisation of the cytoskeleton. Also known as: PCP pathway, Wnt receptor signaling pathway, planar cell polarity pathway, Wnt receptor signalling pathway, planar cell polarity pathway, Wnt-activated signaling pathway, planar cell polarity pathway, planar cell polarity pathway, Wnt-JNK signaling pathway, Wnt-PCP signaling pathway, non-canonical Wnt signaling pathway